{
  "term_id": "GO:0005886",
  "gene": "UniProtKB:Q7Z5H4",
  "gene_name": "Vomeronasal type-1 receptor 5",
  "gene_symbol": "VN1R5",
  "term_label": "plasma membrane"
}